{
  "gene_name": "GTP-binding protein RAD",
  "term_id": "GO:0005246",
  "term_label": "calcium channel regulator activity",
  "gene_symbol": "RRAD",
  "gene": "UniProtKB:P55042"
}